negative regulation of stomatal opening [GO:1902457] (biological process) Relationships: is a type of negative regulation of cellular process [GO:0048523]; is a type of regulation of stomatal opening [GO:1902456]; negatively regulates stomatal opening [GO:1990069] Also known as: down regulation of stomatal opening, down-regulation of stomatal opening, downregulation of stomatal opening, inhibition of stomatal opening Definition: Any process that stops, prevents or reduces the frequency, rate or extent of stomatal opening. References: PMID:23766366 Sources: GOC:TermGenie